{
  "gene_symbol": "KRTAP13-4",
  "term_label": "Unknown cellular component",
  "term_id": "UNKNOWN:0003",
  "gene": "UniProtKB:Q3LI77",
  "gene_name": "Keratin-associated protein 13-4"
}